chromosome passenger complex [GO:0032133] (CC) Also known as: CPC, CPC complex, chromosomal passenger complex References: PMID:16824200, PMID:19570910 Sources: GOC:vw Definition: A eukaryotically conserved protein complex that localizes to kinetochores in early mitosis, the spindle mid-zone in anaphase B and to the telophase midbody. It has been proposed that the passenger complex coordinates various events based on its location to different structures during the course of mitosis. Complex members include the BIR-domain-containing protein Survivin, Aurora kinase, INCENP and Borealin. Relationships: is a type of microtubule associated complex [GO:0005875]